{
  "term_id": "GO:0005829",
  "gene_name": "Golgi phosphoprotein 3",
  "gene": "UniProtKB:Q9H4A6",
  "term_label": "cytosol",
  "gene_symbol": "GOLPH3"
}